{
  "gene_symbol": "CLEC18C",
  "term_label": "extracellular space",
  "term_id": "GO:0005615",
  "gene_name": "C-type lectin domain family 18 member C",
  "gene": "UniProtKB:Q8NCF0"
}